{
  "term_label": "RNA polymerase II cis-regulatory region sequence-specific DNA binding",
  "gene_symbol": "ATF3",
  "term_id": "GO:0000978",
  "gene": "UniProtKB:P18847",
  "gene_name": "Cyclic AMP-dependent transcription factor ATF-3"
}